{
  "term_label": "calmodulin binding",
  "term_id": "GO:0005516",
  "gene_symbol": "UNC13C",
  "gene_name": "Protein unc-13 homolog C",
  "gene": "UniProtKB:Q8NB66"
}